{
  "gene_name": "Protein FRG2-like-1",
  "gene_symbol": "FRG2B",
  "gene": "UniProtKB:Q96QU4",
  "term_label": "Unknown molecular function",
  "term_id": "UNKNOWN:0001"
}